female gamete generation [GO:0007292] (biological process) Definition: Generation of the female gamete; specialised haploid cells produced by meiosis and along with a male gamete takes part in sexual reproduction. Sources: GOC:dph, ISBN:0198506732 Relationships: is a type of gamete generation [GO:0007276] Subtypes: oogenesis [GO:0048477]